{
  "gene_symbol": "MAFG",
  "gene_name": "Transcription factor MafG",
  "term_label": "nucleus",
  "term_id": "GO:0005634",
  "gene": "UniProtKB:O15525"
}